{
  "gene": "UniProtKB:Q08708",
  "gene_name": "CMRF35-like molecule 6",
  "term_label": "transmembrane signaling receptor activity",
  "term_id": "GO:0004888",
  "gene_symbol": "CD300C"
}